{
  "gene": "UniProtKB:Q9UPV9",
  "term_id": "GO:0017022",
  "gene_symbol": "TRAK1",
  "gene_name": "Trafficking kinesin-binding protein 1",
  "term_label": "myosin binding"
}